{
  "gene_symbol": "HSPA1A",
  "gene_name": "Heat shock 70 kDa protein 1A",
  "term_label": "nucleus",
  "term_id": "GO:0005634",
  "gene": "UniProtKB:P0DMV8"
}